{
  "gene_symbol": "SNRPB",
  "gene": "UniProtKB:P14678",
  "term_id": "GO:0070990",
  "term_label": "snRNP binding",
  "gene_name": "Small nuclear ribonucleoprotein-associated proteins B and B'"
}